{
  "term_id": "GO:0045211",
  "term_label": "postsynaptic membrane",
  "gene_symbol": "SHISA7",
  "gene": "UniProtKB:A6NL88",
  "gene_name": "Protein shisa-7"
}